plastid chromosome packaging [GO:1900160] (biological process) Relationships: is a type of chromosome organization [GO:0051276]; occurs in plastid [GO:0009536] References: PMID:12081370 Sources: GOC:TermGenie, GOC:emb Definition: A process in which plastidial DNA and associated proteins organize into a compact, orderly structure. Also known as: DNA organisation in plastid, DNA organization in plastid, plastid DNA packaging, plastidial DNA packaging